{
  "gene_name": "Overexpressed in colon carcinoma 1 protein",
  "gene_symbol": "OCC1",
  "term_label": "Unknown biological process",
  "gene": "UniProtKB:Q8TAD7",
  "term_id": "UNKNOWN:0002"
}